{
  "term_label": "negative regulation of IRE1-mediated unfolded protein response",
  "gene_name": "DDRGK domain-containing protein 1",
  "gene_symbol": "DDRGK1",
  "term_id": "GO:1903895",
  "gene": "UniProtKB:Q96HY6"
}